{
  "gene_name": "MARCO-like protein",
  "term_label": "Unknown cellular component",
  "gene_symbol": "MARCOL",
  "term_id": "UNKNOWN:0003",
  "gene": "UniProtKB:A0A1B0GUY1"
}